phycocyanobilin biosynthetic process [GO:0140609] (biological process) Also known as: phycocyanobilin biosynthesis References: PMID:23345435 Relationships: is_a tetrapyrrole biosynthetic process [GO:0033014] Definition: The chemical reactions or pathway resulting in the formation of phycocyanobilin, which involves the oxidative cleavage of heme by a heme oxygenase (HO) to form biliverdin IX alpha. Biliverdin IX alpha is subsequently converted to phycocyanobilin by a ferredoxin-dependent oxidoreductase (PCYA).